{
  "gene_name": "Synaptosomal-associated protein 29",
  "gene_symbol": "SNAP29",
  "term_label": "plasma membrane",
  "gene": "UniProtKB:O95721",
  "term_id": "GO:0005886"
}